{
  "gene_name": "X-linked retinitis pigmentosa GTPase regulator-interacting protein 1",
  "term_id": "GO:0032391",
  "gene": "UniProtKB:Q96KN7",
  "gene_symbol": "RPGRIP1",
  "term_label": "photoreceptor connecting cilium"
}